{
  "term_label": "Unknown molecular function",
  "gene_name": "NADH dehydrogenase [ubiquinone] 1 alpha subcomplex assembly factor 3",
  "term_id": "UNKNOWN:0001",
  "gene": "UniProtKB:Q9BU61",
  "gene_symbol": "NDUFAF3"
}